neuron projection retraction [GO:0106028] (biological process) Also known as: neuron projection disassembly Relationships: is_a neuron projection organization [GO:0106027] Definition: The organization process which results in the disassembly (either partial or complete) of constituent parts of a neuron projection. A neuron projection is a prolongation or process extending from a nerve cell, e.g. an axon or dendrite. References: PMID:11585923 Sources: GOC:aruk, GOC:bc